{
  "gene": "UniProtKB:Q5TEA3",
  "term_id": "UNKNOWN:0003",
  "gene_symbol": "DNAAF9",
  "term_label": "Unknown cellular component",
  "gene_name": "Dynein axonemal assembly factor 9"
}